{
  "gene_symbol": "EPB41",
  "gene_name": "Protein 4.1",
  "gene": "UniProtKB:P11171",
  "term_label": "Unknown molecular function",
  "term_id": "UNKNOWN:0001"
}